{
  "gene_name": "HERV-H LTR-associating protein 2",
  "gene_symbol": "HHLA2",
  "gene": "UniProtKB:Q9UM44",
  "term_id": "GO:0050852",
  "term_label": "T cell receptor signaling pathway"
}